mannosylglycerate synthase activity [GO:0102921] (molecular function) Relationships: is a type of hexosyltransferase activity [GO:0016758] Definition: Catalysis of the reaction: GDP-alpha-D-mannose + D-glycerate = H+ + 2-(alpha-D-mannosyl)-D-glycerate + GDP. Sources: EC:2.4.1.269, GOC:pz